{
  "term_id": "UNKNOWN:0003",
  "gene_name": "Keratin-associated protein 6-2",
  "gene_symbol": "KRTAP6-2",
  "gene": "UniProtKB:Q3LI66",
  "term_label": "Unknown cellular component"
}